{
  "gene_name": "Tectonic-1",
  "gene": "UniProtKB:Q2MV58",
  "term_id": "GO:0036038",
  "gene_symbol": "TCTN1",
  "term_label": "MKS complex"
}